{
  "gene": "UniProtKB:Q9HC38",
  "term_label": "Unknown molecular function",
  "gene_name": "Glyoxalase domain-containing protein 4",
  "gene_symbol": "GLOD4",
  "term_id": "UNKNOWN:0001"
}